{
  "gene_name": "BRISC and BRCA1-A complex member 1",
  "gene": "UniProtKB:Q9NWV8",
  "gene_symbol": "BABAM1",
  "term_label": "BRCA1-A complex",
  "term_id": "GO:0070531"
}